morula formation [GO:0140001] (biological process) Definition: The initial formation of a spherical embryonic mass of blastomeres formed before the blastula and resulting from cleavage of the fertilized ovum. Relationships: is a type of GO:0048646 References: PMID:37935903, PMID:38386558, PMID:39361745